{
  "term_id": "GO:0006357",
  "gene": "UniProtKB:Q01094",
  "gene_name": "Transcription factor E2F1",
  "term_label": "regulation of transcription by RNA polymerase II",
  "gene_symbol": "E2F1"
}